interleukin-24 binding [GO:0045510] (molecular function) Sources: GOC:go_curators Also known as: IL-24 binding Definition: Binding to interleukin-24. Relationships: is a type of cytokine binding [GO:0019955]